peptidoglycan cross-bridge peptide endopeptidase activity [GO:0061787] (MF) References: PMID:22748813 Sources: GOC:dph, GOC:jh Also known as: lysostaphin activity Relationships: is a type of GO:0061785 Definition: A peptidoglycan endopeptidase activity that acts on a peptidoglycan cross-bridge.